{
  "term_label": "nucleus",
  "gene": "UniProtKB:P22736",
  "gene_symbol": "NR4A1",
  "term_id": "GO:0005634",
  "gene_name": "Nuclear receptor subfamily 4 group A member 1"
}